positive regulation of smooth muscle cell-matrix adhesion [GO:1905609] (biological process) References: PMID:14970114 Sources: GOC:TermGenie, GO_REF:0000058 Definition: Any process that activates or increases the frequency, rate or extent of smooth muscle cell-matrix adhesion. Relationships: is a type of positive regulation of cell-matrix adhesion [GO:0001954]; is a type of regulation of smooth muscle cell-matrix adhesion [GO:2000097]; positively regulates smooth muscle cell-matrix adhesion [GO:0061302] Also known as: up regulation of smooth muscle cell-matrix adhesion, up-regulation of smooth muscle cell-matrix adhesion, upregulation of smooth muscle cell-matrix adhesion, activation of smooth muscle cell-matrix adhesion